{
  "term_label": "cytosol",
  "gene_symbol": "RPEL1",
  "gene_name": "Ribulose-phosphate 3-epimerase-like protein 1",
  "term_id": "GO:0005829",
  "gene": "UniProtKB:Q2QD12"
}